{
  "term_label": "response to lipopolysaccharide",
  "gene_name": "Nitric oxide synthase 1",
  "gene_symbol": "NOS1",
  "gene": "UniProtKB:P29475",
  "term_id": "GO:0032496"
}